complement component C3b binding [GO:0001851] (molecular function) Definition: Binding to a C3b product of the complement cascade. Sources: GOC:add, ISBN:0781735149 Relationships: is a type of opsonin binding [GO:0001846]; is a type of GO:0001848